ammonia-lyase activity [GO:0016841] (MF) Definition: Catalysis of the release of ammonia by the cleavage of a carbon-nitrogen bond or the reverse reaction with ammonia as a substrate. Relationships: is a type of carbon-nitrogen lyase activity [GO:0016840] Subtypes: L-serine ammonia-lyase activity [GO:0003941], histidine ammonia-lyase activity [GO:0004397], threonine deaminase activity [GO:0004794], ornithine cyclodeaminase activity [GO:0008473], GO:0008721, aspartate ammonia-lyase activity [GO:0008797], diaminopropionate ammonia-lyase activity [GO:0008838], ethanolamine ammonia-lyase activity [GO:0008851], formimidoyltetrahydrofolate cyclodeaminase activity [GO:0030412], threo-3-hydroxyaspartate ammonia-lyase activity [GO:0030848], 7,8-didemethyl-8-hydroxy-5-deazariboflavin synthase activity [GO:0044689], GO:0045548, erythro-3-hydroxyaspartate ammonia-lyase activity [GO:0047447], GO:0047459, GO:0047698, carbamoyl-serine ammonia-lyase activity [GO:0047766], glucosaminate ammonia-lyase activity [GO:0047930], GO:0050096, GO:0050283, tyrosine ammonia-lyase activity [GO:0052883], ADP-riboxanase activity [GO:0140740] Sources: GOC:krc